{
  "term_label": "phagocytic vesicle",
  "gene_name": "Rab11 family-interacting protein 5",
  "term_id": "GO:0045335",
  "gene": "UniProtKB:Q9BXF6",
  "gene_symbol": "RAB11FIP5"
}